negative regulation of heptadecane biosynthetic process [GO:1900897] (biological process) Relationships: is a type of regulation of heptadecane biosynthetic process [GO:1900896]; is a type of negative regulation of alkane biosynthetic process [GO:1901578]; negatively regulates heptadecane biosynthetic process [GO:1900636] Also known as: down regulation of heptadecane biosynthetic process, down-regulation of heptadecane biosynthetic process, downregulation of heptadecane biosynthetic process, inhibition of heptadecane anabolism, inhibition of heptadecane biosynthesis, inhibition of heptadecane biosynthetic process, inhibition of heptadecane formation, inhibition of heptadecane synthesis, down regulation of heptadecane anabolism, down regulation of heptadecane biosynthesis, down regulation of heptadecane formation, down regulation of heptadecane synthesis, down-regulation of heptadecane anabolism, down-regulation of heptadecane biosynthesis, down-regulation of heptadecane formation, down-regulation of heptadecane synthesis, downregulation of heptadecane anabolism, downregulation of heptadecane biosynthesis, downregulation of heptadecane formation, downregulation of heptadecane synthesis, negative regulation of heptadecane anabolism, negative regulation of heptadecane biosynthesis, negative regulation of heptadecane formation, negative regulation of heptadecane synthesis Definition: Any process that stops, prevents or reduces the frequency, rate or extent of heptadecane biosynthetic process. Sources: GOC:TermGenie, GOC:mengo_curators